{
  "gene": "UniProtKB:Q8WV28",
  "term_id": "GO:0035556",
  "gene_name": "B-cell linker protein",
  "term_label": "intracellular signal transduction",
  "gene_symbol": "BLNK"
}